{
  "term_id": "UNKNOWN:0001",
  "gene_name": "T cell receptor gamma variable 2",
  "gene": "UniProtKB:A0A075B6R0",
  "gene_symbol": "TRGV2",
  "term_label": "Unknown molecular function"
}